{
  "term_id": "GO:0071526",
  "gene": "UniProtKB:Q99985",
  "term_label": "semaphorin-plexin signaling pathway",
  "gene_symbol": "SEMA3C",
  "gene_name": "Semaphorin-3C"
}